{
  "term_id": "UNKNOWN:0001",
  "gene_symbol": "TAS2R19",
  "gene_name": "Taste receptor type 2 member 19",
  "gene": "UniProtKB:P59542",
  "term_label": "Unknown molecular function"
}